{
  "term_id": "GO:0006260",
  "term_label": "DNA replication",
  "gene_symbol": "RECQL4",
  "gene": "UniProtKB:O94761",
  "gene_name": "ATP-dependent DNA helicase Q4"
}